symbiont-mediated disruption of host antimicrobial peptide activity [GO:0141059] (biological process) Relationships: is a type of symbiont-mediated suppression of host defenses [GO:0044414] Also known as: disruption of host antimicrobial peptide activity References: PMID:16242332, PMID:19015361, PMID:21335044 Definition: Any process in which a symbiont interferes with a host antimicrobial peptide, for example by cleavage or degradation.